{
  "term_id": "UNKNOWN:0002",
  "term_label": "Unknown biological process",
  "gene": "UniProtKB:A6NIY4",
  "gene_name": "Speedy protein E5",
  "gene_symbol": "SPDYE5"
}